{
  "term_label": "neuron projection",
  "gene": "UniProtKB:P50391",
  "gene_symbol": "NPY4R",
  "term_id": "GO:0043005",
  "gene_name": "Neuropeptide Y receptor type 4"
}